regulation of skeletal muscle contraction by regulation of release of sequestered calcium ion [GO:0014809] (biological process) Subtypes: positive regulation of skeletal muscle contraction by regulation of release of sequestered calcium ion [GO:0014810], negative regulation of skeletal muscle contraction by regulation of release of sequestered calcium ion [GO:0014811] Definition: Any process that modulates the frequency, rate or extent of skeletal muscle contraction via the regulation of the release of sequestered calcium ion by sarcoplasmic reticulum into cytosol. The sarcoplasmic reticulum is the endoplasmic reticulum of striated muscle, specialised for the sequestration of calcium ions that are released upon receipt of a signal relayed by the T tubules from the neuromuscular junction. Relationships: is a type of regulation of release of sequestered calcium ion into cytosol by sarcoplasmic reticulum [GO:0010880]; is a type of regulation of skeletal muscle contraction by calcium ion signaling [GO:0014722] Sources: GOC:mtg_muscle